{
  "gene": "UniProtKB:P78524",
  "gene_symbol": "DENND2B",
  "term_id": "UNKNOWN:0001",
  "gene_name": "DENN domain-containing protein 2B",
  "term_label": "Unknown molecular function"
}